{
  "gene": "UniProtKB:O43612",
  "term_id": "GO:0031772",
  "gene_name": "Hypocretin neuropeptide precursor",
  "term_label": "type 2 orexin receptor binding",
  "gene_symbol": "HCRT"
}